pigment granule localization [GO:0051875] (BP) Subtypes: GO:0032400, pigment granule transport [GO:0051904] Relationships: is a type of GO:0051648; is part of cellular pigmentation [GO:0033059] Also known as: pigment granule localisation Sources: GOC:ai Definition: Any process in which a pigment granule is transported to, and/or maintained in, a specific location within the cell.